organelle envelope [GO:0031967] (cellular component) Definition: A double membrane structure enclosing an organelle, including two lipid bilayers and the region between them. In some cases, an organelle envelope may have more than two membranes. Sources: GOC:mah, GOC:pz Relationships: is a type of cellular anatomical structure [GO:0110165]; is part of GO:0043227; is part of intracellular organelle [GO:0043229] Subtypes: GO:0005635, GO:0005740, plastid envelope [GO:0009526], GO:0070732